{
  "term_id": "GO:0034388",
  "gene_symbol": "UTP18",
  "term_label": "Pwp2p-containing subcomplex of 90S preribosome",
  "gene": "UniProtKB:Q9Y5J1",
  "gene_name": "U3 small nucleolar RNA-associated protein 18 homolog"
}